{
  "term_id": "GO:0005516",
  "term_label": "calmodulin binding",
  "gene": "UniProtKB:Q13576",
  "gene_name": "Ras GTPase-activating-like protein IQGAP2",
  "gene_symbol": "IQGAP2"
}